{
  "gene_symbol": "STAT5B",
  "gene_name": "Signal transducer and activator of transcription 5B",
  "gene": "UniProtKB:P51692",
  "term_id": "GO:0006357",
  "term_label": "regulation of transcription by RNA polymerase II"
}